{
  "gene_name": "T cell receptor beta variable 5-6",
  "gene": "UniProtKB:A0A599",
  "gene_symbol": "TRBV5-6",
  "term_label": "cell surface receptor signaling pathway",
  "term_id": "GO:0007166"
}